{
  "term_id": "GO:0005769",
  "term_label": "early endosome",
  "gene_name": "E3 ubiquitin-protein ligase NEURL1B",
  "gene": "UniProtKB:A8MQ27",
  "gene_symbol": "NEURL1B"
}